{
  "gene_symbol": "FBXO33",
  "gene": "UniProtKB:Q7Z6M2",
  "term_id": "UNKNOWN:0003",
  "gene_name": "F-box only protein 33",
  "term_label": "Unknown cellular component"
}